{
  "term_id": "GO:0005737",
  "gene_name": "Fibroblast growth factor 3",
  "gene_symbol": "FGF3",
  "gene": "UniProtKB:P11487",
  "term_label": "cytoplasm"
}